L-propargylglycine synthase activity [GO:0062144] (molecular function) Relationships: is a type of carbon-halide lyase activity [GO:0016848] References: PMID:30867596 Sources: RHEA:59892 Definition: Catalysis of the reaction: L-2-amino-4-chloropent-4-enoate = chloride + H+ + L-propargylglycine.